tensidol B catabolic process [GO:1900607] (biological process) Relationships: is a type of GO:0042182; is a type of amide metabolic process [GO:0043603]; is a type of GO:0046395; is a type of secondary metabolite catabolic process [GO:0090487] Definition: The chemical reactions and pathways resulting in the breakdown of tensidol B. Sources: GOC:TermGenie, GOC:di Also known as: tensidol B breakdown, tensidol B catabolism, tensidol B degradation